venom-mediated vasodilation via suppression of angiotensin maturation [GO:0140166] (biological process) References: PMID:31370142 Also known as: venom-mediated vasodilation mediated by inhibition of angiotensin-converting enzyme, venom-mediated vasodilation through perturbation of angiotensin maturation Relationships: is a type of venom-mediated perturbation of signal transduction [GO:0044509]; is_a venom-mediated vasodilation [GO:0044551] Definition: A process in which an organism initiates, promotes, or enhances vasodilation via the action of a venom that prevents angiotensin maturation, concomittantly reducing blood pressure in the bitten/stung organism.